{
  "gene_name": "Immunoglobulin kappa variable 1-16",
  "term_label": "immune response",
  "term_id": "GO:0006955",
  "gene_symbol": "IGKV1-16",
  "gene": "UniProtKB:P04430"
}